{
  "gene": "UniProtKB:P0DPD8",
  "gene_name": "EEF1AKMT4-ECE2 readthrough transcript protein",
  "term_id": "GO:0016485",
  "term_label": "protein processing",
  "gene_symbol": "EEF1AKMT4-ECE2"
}